high molecular weight B cell growth factor receptor binding [GO:0030372] (molecular function) Relationships: is a type of growth factor receptor binding [GO:0070851] Definition: Binding to a high molecular weight B cell growth factor receptor. Also known as: high molecular weight B lymphocyte growth factor receptor binding, high molecular weight B-cell growth factor receptor binding, high molecular weight B-lymphocyte growth factor receptor binding, high molecular weight B cell growth factor receptor ligand Sources: GOC:ai